{
  "term_label": "Unknown molecular function",
  "term_id": "UNKNOWN:0001",
  "gene_symbol": "TRBV2",
  "gene": "UniProtKB:A0A1B0GX68",
  "gene_name": "T cell receptor beta variable 2"
}